response to interleukin-15 [GO:0070672] (biological process) Also known as: response to IL-15 Relationships: is a type of response to cytokine [GO:0034097] Sources: GOC:mah Definition: Any process that results in a change in state or activity of a cell or an organism (in terms of movement, secretion, enzyme production, gene expression, etc.) as a result of an interleukin-15 stimulus. Subtypes: cellular response to interleukin-15 [GO:0071350]